{
  "term_id": "GO:0002286",
  "gene": "UniProtKB:P05014",
  "gene_symbol": "IFNA4",
  "term_label": "T cell activation involved in immune response",
  "gene_name": "Interferon alpha-4"
}